{
  "term_label": "immunoglobulin mediated immune response",
  "gene": "UniProtKB:A0A0C4DH30",
  "term_id": "GO:0016064",
  "gene_symbol": "IGHV3-16",
  "gene_name": "Probable non-functional immunoglobulin heavy variable 3-16"
}